{
  "term_label": "Unknown cellular component",
  "gene": "UniProtKB:Q9Y6P5",
  "term_id": "UNKNOWN:0003",
  "gene_symbol": "SESN1",
  "gene_name": "Sestrin-1"
}